{
  "term_label": "DNA-templated transcription initiation",
  "gene": "UniProtKB:P20226",
  "gene_symbol": "TBP",
  "term_id": "GO:0006352",
  "gene_name": "TATA-box-binding protein"
}